UDP-L-arabinose metabolic process [GO:0033356] (BP) Subtypes: UDP-L-arabinose biosynthetic process [GO:0033358] Definition: The chemical reactions and pathways involving UDP-L-arabinose, uridinediphosphoarabinose, a substance composed of arabinose in glycosidic linkage with uridine diphosphate. Relationships: is a type of nucleotide-sugar metabolic process [GO:0009225] Sources: GOC:mah Also known as: UDP-L-arabinose metabolism